inositol pentakisphosphate phosphatase activity [GO:0052827] (molecular function) Sources: GOC:bf Subtypes: inositol-1,3,4,5,6-pentakisphosphate 3-phosphatase activity [GO:0030351], inositol-1,3,4,5,6-pentakisphosphate 1-phosphatase activity [GO:0052825], inositol-1,2,4,5,6-pentakisphosphate 5-phosphatase activity [GO:1990651] Relationships: is a type of inositol phosphate phosphatase activity [GO:0052745] Definition: Catalysis of the reaction: myo-inositol pentakisphosphate + H2O = myo-inositol tetrakisphosphate + phosphate.